ephrin receptor activity [GO:0005003] (molecular function) Subtypes: GPI-linked ephrin receptor activity [GO:0005004], transmembrane-ephrin receptor activity [GO:0005005] Also known as: Eph receptor activity References: PMID:9530499 Sources: GOC:mah Relationships: is_a GO:0004714; is part of ephrin receptor signaling pathway [GO:0048013] Definition: Combining with an ephrin receptor ligand to initiate a change in cell activity.